{
  "gene_symbol": "DCTN5",
  "term_id": "GO:0005869",
  "gene": "UniProtKB:Q9BTE1",
  "term_label": "dynactin complex",
  "gene_name": "Dynactin subunit 5"
}